{
  "gene": "UniProtKB:Q15399",
  "gene_symbol": "TLR1",
  "gene_name": "Toll-like receptor 1",
  "term_label": "Toll-like receptor 1-Toll-like receptor 2 protein complex",
  "term_id": "GO:0035354"
}